{
  "term_label": "SCF ubiquitin ligase complex",
  "gene": "UniProtKB:Q13309",
  "gene_name": "S-phase kinase-associated protein 2",
  "term_id": "GO:0019005",
  "gene_symbol": "SKP2"
}